{
  "gene_symbol": "RSC1A1",
  "gene": "UniProtKB:Q92681",
  "gene_name": "Regulatory solute carrier protein family 1 member 1",
  "term_id": "UNKNOWN:0001",
  "term_label": "Unknown molecular function"
}